{
  "term_id": "GO:0007155",
  "gene_name": "Protocadherin-11 X-linked",
  "gene_symbol": "PCDH11X",
  "gene": "UniProtKB:Q9BZA7",
  "term_label": "cell adhesion"
}